positive regulation of primary cell septum biogenesis [GO:1905758] (biological process) Definition: Any process that activates or increases the frequency, rate or extent of primary cell septum biogenesis. References: PMID:27898700 Sources: GOC:TermGenie, GO_REF:0000058 Relationships: is a type of positive regulation of cellular component biogenesis [GO:0044089]; is a type of positive regulation of mitotic cytokinetic process [GO:1903438]; is a type of GO:1905756; positively regulates primary cell septum biogenesis [GO:0031671]